response to ionizing radiation [GO:0010212] (biological process) Also known as: response to ionising radiation, response to ionizing radiation stimulus Definition: Any process that results in a change in state or activity of a cell or an organism (in terms of movement, secretion, enzyme production, gene expression, etc.) as a result of a ionizing radiation stimulus. Ionizing radiation is radiation with sufficient energy to remove electrons from atoms and may arise from spontaneous decay of unstable isotopes, resulting in alpha and beta particles and gamma rays. Ionizing radiation also includes X-rays. Subtypes: GO:0010165, response to gamma radiation [GO:0010332], cellular response to ionizing radiation [GO:0071479] Relationships: is a type of response to radiation [GO:0009314] References: PMID:12509526